{
  "term_label": "nuclear pore",
  "gene_symbol": "NUP153",
  "term_id": "GO:0005643",
  "gene_name": "Nuclear pore complex protein Nup153",
  "gene": "UniProtKB:P49790"
}